regulation of response to propan-1-ol [GO:1901445] (biological process) Relationships: is a type of regulation of response to alcohol [GO:1901419]; regulates response to propan-1-ol [GO:1901427] Sources: GOC:TermGenie, GOC:mengo_curators Subtypes: GO:1901446, positive regulation of response to propan-1-ol [GO:1901447] Definition: Any process that modulates the frequency, rate or extent of response to propan-1-ol.